{
  "gene": "UniProtKB:Q96P69",
  "gene_symbol": "GPR78",
  "term_label": "adenylate cyclase-activating G protein-coupled receptor signaling pathway",
  "term_id": "GO:0007189",
  "gene_name": "G-protein coupled receptor 78"
}